negative regulation of isotype switching to IgD isotypes [GO:0048300] (biological process) Definition: Any process that stops, prevents, or reduces the frequency, rate or extent of isotype switching to IgD isotypes. Relationships: is a type of negative regulation of isotype switching [GO:0045829]; is a type of regulation of isotype switching to IgD isotypes [GO:0048299]; negatively regulates isotype switching to IgD isotypes [GO:0048292] Also known as: down regulation of isotype switching to IgD isotypes, down-regulation of isotype switching to IgD isotypes, downregulation of isotype switching to IgD isotypes, negative regulation of class switch recombination to IgD isotypes, negative regulation of class switching to IgD isotypes, negative regulation of isotype switch recombination to IgD isotypes, inhibition of isotype switching to IgD isotypes Sources: GOC:jid